{
  "gene": "UniProtKB:Q8NE09",
  "term_label": "nucleus",
  "gene_name": "Regulator of G-protein signaling 22",
  "term_id": "GO:0005634",
  "gene_symbol": "RGS22"
}